{
  "gene": "UniProtKB:P33991",
  "gene_symbol": "MCM4",
  "term_id": "GO:0000727",
  "term_label": "double-strand break repair via break-induced replication",
  "gene_name": "DNA replication licensing factor MCM4"
}